response to methylglyoxal [GO:0051595] (biological process) Sources: GOC:ai Definition: Any process that results in a change in state or activity of a cell or an organism (in terms of movement, secretion, enzyme production, gene expression, etc.) as a result of a methylglyoxal stimulus. Methylglyoxal is a 2-oxoaldehyde derived from propanal. Relationships: is a type of response to ketone [GO:1901654] Also known as: response to pyruvaldehyde Subtypes: cellular response to methylglyoxal [GO:0097238]